sulfur amino acid biosynthetic process [GO:0000097] (biological process) Also known as: sulfur amino acid anabolism, sulfur amino acid biosynthesis, sulfur amino acid formation, sulfur amino acid synthesis, sulphur amino acid biosynthesis, sulphur amino acid biosynthetic process Definition: The chemical reactions and pathways resulting in the formation of amino acids containing sulfur, comprising cysteine, methionine and selenocysteine. Sources: GOC:ai Relationships: is_a GO:0000096; is a type of sulfur compound biosynthetic process [GO:0044272]; is a type of GO:0046394 Subtypes: methionine biosynthetic process [GO:0009086], cysteine biosynthetic process [GO:0019344], ergothioneine biosynthetic process [GO:0052699], homocysteine biosynthetic process [GO:0071268]